cordyol C catabolic process [GO:1900798] (biological process) Definition: The chemical reactions and pathways resulting in the breakdown of cordyol C. Relationships: is a type of catechol-containing compound catabolic process [GO:0019614]; is a type of GO:0090487; is a type of cordyol C metabolic process [GO:1900797]; is a type of ether catabolic process [GO:1901502] Also known as: cordyol C breakdown, cordyol C catabolism, cordyol C degradation Sources: GOC:TermGenie, GOC:di